{
  "gene_name": "WD and tetratricopeptide repeats protein 1",
  "term_label": "Unknown molecular function",
  "term_id": "UNKNOWN:0001",
  "gene": "UniProtKB:Q8N5D0",
  "gene_symbol": "WDTC1"
}